{
  "term_label": "cysteine-type endopeptidase inhibitor activity involved in apoptotic process",
  "gene_name": "E3 ubiquitin-protein ligase XIAP",
  "gene_symbol": "XIAP",
  "gene": "UniProtKB:P98170",
  "term_id": "GO:0043027"
}